{
  "gene_symbol": "ADGRA2",
  "term_label": "Unknown molecular function",
  "gene_name": "Adhesion G protein-coupled receptor A2",
  "term_id": "UNKNOWN:0001",
  "gene": "UniProtKB:Q96PE1"
}